arthrospore formation [GO:0034298] (biological process) Also known as: arthroconidium formation Sources: GOC:mah Definition: The formation of conidia by the conversion of a pre-existing hypha. An arthrospore is produced by the last cell on a hypha breaking off and dispersing. Usually the walls thicken and the cell(s) separates before swelling of each spore. Sometimes further septa form in each cell prior to disarticulation. Relationships: is_a conidium formation [GO:0048315]; is a type of anatomical structure formation involved in morphogenesis [GO:0048646]